{
  "gene": "UniProtKB:Q53S08",
  "term_id": "GO:0005794",
  "gene_name": "Ras-related protein Rab-6D",
  "term_label": "Golgi apparatus",
  "gene_symbol": "RAB6D"
}